regulation of erythrocyte aggregation [GO:0034118] (biological process) Subtypes: negative regulation of erythrocyte aggregation [GO:0034119], positive regulation of erythrocyte aggregation [GO:0034120] Also known as: regulation of RBC aggregation, regulation of red blood cell aggregation Sources: GOC:add Definition: Any process that modulates the frequency, rate, or extent of erythrocyte aggregation. Relationships: is a type of regulation of homotypic cell-cell adhesion [GO:0034110]; regulates erythrocyte aggregation [GO:0034117]